phosphatidylcholine acyl-chain remodeling [GO:0036151] (biological process) Also known as: phosphatidylcholine acyl-chain remodelling References: PMID:18195019, PMID:18458083 Sources: GOC:mw Relationships: is a type of phosphatidylcholine metabolic process [GO:0046470] Definition: Remodeling the acyl chains of phosphatidylcholine, through sequential deacylation and re-acylation reactions, to generate phosphatidylcholine containing different types of fatty acid acyl chains.